vesicle-mediated transport in synapse [GO:0099003] (biological process) Sources: GOC:dos Relationships: is a type of GO:0016192; occurs in synapse [GO:0045202] Definition: Any vesicle-mediated transport that occurs in a synapse. Subtypes: GO:0016079, synaptic vesicle budding from endosome [GO:0016182], synaptic vesicle cycle [GO:0099504], endocytosed synaptic vesicle processing via endosome [GO:0099592], presynaptic endocytosis [GO:0140238], postsynaptic endocytosis [GO:0140239], postsynaptic dense core vesicle exocytosis [GO:0150038]